mitochondrial calcium ion transmembrane transport [GO:0006851] (BP) Subtypes: GO:0036444, calcium export from the mitochondrion [GO:0099093] Definition: The process in which a calcium ion (Ca2+) is transported across a mitochondrial membrane, into or out of the mitochondrion. Sources: GOC:ai Also known as: mitochondrial calcium transport Relationships: is a type of calcium ion transmembrane transport [GO:0070588]